{
  "term_id": "GO:0005634",
  "gene_name": "Akirin-1",
  "term_label": "nucleus",
  "gene": "UniProtKB:Q9H9L7",
  "gene_symbol": "AKIRIN1"
}